{
  "term_id": "GO:0000978",
  "gene": "UniProtKB:Q8IYN0",
  "gene_symbol": "ZNF100",
  "term_label": "RNA polymerase II cis-regulatory region sequence-specific DNA binding",
  "gene_name": "Zinc finger protein 100"
}